septate junction assembly [GO:0019991] (biological process) Subtypes: smooth septate junction assembly [GO:0090528] Relationships: is a type of tight junction assembly [GO:0120192]; is part of apical junction assembly [GO:0043297] References: PMID:5272312 Sources: GOC:ai Definition: The assembly of a septate junction, an intercellular junction found in invertebrate epithelia that is characterized by a ladder like appearance in electron micrographs and thought to provide structural strength and to provide a barrier to diffusion of solutes through the intercellular space.